{
  "gene_symbol": "TRPC3",
  "gene_name": "Short transient receptor potential channel 3",
  "term_id": "GO:0070588",
  "gene": "UniProtKB:Q13507",
  "term_label": "calcium ion transmembrane transport"
}